regulation of neuron remodeling [GO:1904799] (biological process) Definition: Any process that modulates the frequency, rate or extent of neuron remodeling. Note: cyy-1 in C. Elegans (P34624) in PMID:21609829 (inferred from mutant phenotype) Also known as: regulation of neuron remodelling, regulation of neuronal remodeling, regulation of axon pruning References: PMID:21609829 Sources: GOC:TermGenie, GO_REF:0000058 Subtypes: negative regulation of neuron remodeling [GO:1904800], GO:1904801 Relationships: is a type of regulation of neuron maturation [GO:0014041]; regulates neuron remodeling [GO:0016322]